{
  "term_id": "UNKNOWN:0002",
  "gene_symbol": "FAM219B",
  "gene_name": "Protein FAM219B",
  "term_label": "Unknown biological process",
  "gene": "UniProtKB:Q5XKK7"
}